{
  "term_label": "extracellular space",
  "gene": "UniProtKB:Q8IUB2",
  "term_id": "GO:0005615",
  "gene_name": "WAP four-disulfide core domain protein 3",
  "gene_symbol": "WFDC3"
}